{
  "gene_symbol": "GOLGA8G",
  "gene_name": "Putative golgin subfamily A member 8F_8G",
  "term_label": "Unknown cellular component",
  "term_id": "UNKNOWN:0003",
  "gene": "UniProtKB:Q08AF8"
}